response to cytarabine [GO:0097331] (biological process) Definition: Any process that results in a change in state or activity of a cell or an organism (in terms of movement, secretion, enzyme production, gene expression, etc.) as a result of a cytarabine stimulus. Relationships: is a type of GO:1901698; is a type of response to glycoside [GO:1903416] Sources: GOC:pr